{
  "gene_symbol": "ZDHHC2",
  "term_id": "GO:0007416",
  "term_label": "synapse assembly",
  "gene_name": "Palmitoyltransferase ZDHHC2",
  "gene": "UniProtKB:Q9UIJ5"
}